{
  "term_id": "UNKNOWN:0003",
  "term_label": "Unknown cellular component",
  "gene_name": "Aryl-hydrocarbon-interacting protein-like 1",
  "gene_symbol": "AIPL1",
  "gene": "UniProtKB:Q9NZN9"
}